{
  "gene_name": "Apoptosis regulator BAX",
  "term_id": "GO:0015267",
  "gene": "UniProtKB:Q07812",
  "gene_symbol": "BAX",
  "term_label": "channel activity"
}